{
  "term_id": "GO:0016279",
  "gene_name": "EEF1A lysine methyltransferase 3",
  "gene_symbol": "EEF1AKMT3",
  "term_label": "protein-lysine N-methyltransferase activity",
  "gene": "UniProtKB:Q96AZ1"
}